{
  "gene": "UniProtKB:Q96GG9",
  "term_id": "GO:0097602",
  "gene_name": "DCN1-like protein 1",
  "gene_symbol": "DCUN1D1",
  "term_label": "cullin family protein binding"
}